{
  "gene_name": "Zinc finger protein 570",
  "term_label": "nucleus",
  "term_id": "GO:0005634",
  "gene_symbol": "ZNF570",
  "gene": "UniProtKB:Q96NI8"
}